{
  "term_label": "insulin-like growth factor receptor binding",
  "gene": "UniProtKB:Q5JWF2",
  "gene_symbol": "GNAS",
  "term_id": "GO:0005159",
  "gene_name": "Guanine nucleotide-binding protein G(s) subunit alpha isoforms XLas"
}